{
  "gene_symbol": "MAP7",
  "gene_name": "Ensconsin",
  "term_id": "GO:0015630",
  "term_label": "microtubule cytoskeleton",
  "gene": "UniProtKB:Q14244"
}